xylogalacturonan metabolic process [GO:0010398] (biological process) Also known as: xylogalacturonan metabolism Sources: GOC:tair_curators Definition: The chemical reactions and pathways involving xylogalacturonan, a pectin characterized by a backbone of alpha-(1->4)-linked D-galacturonic acid residues substituted on C-3 with beta-D-xylopyranose residues. Relationships: is a type of galacturonan metabolic process [GO:0010393]